{
  "term_label": "structural constituent of cytoskeleton",
  "gene": "UniProtKB:P61160",
  "term_id": "GO:0005200",
  "gene_symbol": "ACTR2",
  "gene_name": "Actin-related protein 2"
}